{
  "gene_symbol": "SH3GLB1",
  "term_id": "GO:0006897",
  "gene": "UniProtKB:Q9Y371",
  "term_label": "endocytosis",
  "gene_name": "Endophilin-B1"
}